{
  "gene_name": "Neuronal acetylcholine receptor subunit alpha-9",
  "gene": "UniProtKB:Q9UGM1",
  "gene_symbol": "CHRNA9",
  "term_label": "monoatomic ion transmembrane transport",
  "term_id": "GO:0034220"
}